{
  "gene_symbol": "PERM1",
  "gene_name": "PGC-1 and ERR-induced regulator in muscle protein 1",
  "term_id": "GO:0005634",
  "term_label": "nucleus",
  "gene": "UniProtKB:Q5SV97"
}